{
  "term_label": "protein-N-terminal amino-acid acetyltransferase activity",
  "gene_name": "N-alpha-acetyltransferase 60",
  "term_id": "GO:0004596",
  "gene": "UniProtKB:Q9H7X0",
  "gene_symbol": "NAA60"
}